{
  "gene": "UniProtKB:Q86SJ6",
  "term_id": "GO:0098609",
  "gene_symbol": "DSG4",
  "term_label": "cell-cell adhesion",
  "gene_name": "Desmoglein-4"
}